{
  "gene_name": "COMM domain-containing protein 10",
  "gene_symbol": "COMMD10",
  "term_id": "UNKNOWN:0003",
  "gene": "UniProtKB:Q9Y6G5",
  "term_label": "Unknown cellular component"
}